regulation of vascular associated smooth muscle cell migration [GO:1904752] (biological process) Definition: Any process that modulates the frequency, rate or extent of vascular associated smooth muscle cell migration. References: PMID:20693317 Sources: GOC:BHF, GOC:BHF_miRNA, GOC:TermGenie, GOC:rph, GO_REF:0000058 Also known as: regulation of vascular smooth muscle cell migration Relationships: is a type of regulation of smooth muscle cell migration [GO:0014910]; regulates GO:1904738 Subtypes: negative regulation of vascular associated smooth muscle cell migration [GO:1904753], positive regulation of vascular associated smooth muscle cell migration [GO:1904754]